{
  "term_id": "GO:0043066",
  "gene_symbol": "CRYAB",
  "gene": "UniProtKB:P02511",
  "gene_name": "Alpha-crystallin B chain",
  "term_label": "negative regulation of apoptotic process"
}